{
  "gene_symbol": "TRMT9B",
  "gene": "UniProtKB:Q9P272",
  "term_id": "GO:0005737",
  "term_label": "cytoplasm",
  "gene_name": "Probable tRNA methyltransferase 9B"
}